{
  "gene": "UniProtKB:Q07507",
  "gene_name": "Dermatopontin",
  "term_id": "UNKNOWN:0003",
  "gene_symbol": "DPT",
  "term_label": "Unknown cellular component"
}